{
  "gene": "UniProtKB:P01615",
  "gene_symbol": "IGKV2D-28",
  "term_id": "UNKNOWN:0001",
  "gene_name": "Immunoglobulin kappa variable 2D-28",
  "term_label": "Unknown molecular function"
}